8-hydroxyfuranocoumarin 8-O-methyltransferase activity [GO:0030753] (molecular function) Relationships: is a type of S-adenosylmethionine-dependent methyltransferase activity [GO:0008757] Also known as: xanthotoxol O-methyltransferase activity, S-adenosyl-L-methionine:8-hydroxyfuranocoumarin 8-O-methyltransferase activity, S-adenosyl-L-methionine:8-hydroxyfurocoumarin 8-O-methyltransferase activity, S-adenosyl-L-methionine:xanthotoxol O-methyltransferase activity, XMT activity, furanocoumarin 8-O-methyl-transferase activity, furanocoumarin 8-methyltransferase activity, xanthotoxol 8-O-methyltransferase activity, xanthotoxol methyltransferase activity Sources: EC:2.1.1.70 Definition: Catalysis of the reaction: S-adenosyl-L-methionine + xanthotoxol = S-adenosyl-L-homocysteine + xanthotoxin. Xanthotoxol is also known as 8-hydroxyfuranocoumarin and xanthotoxin as 8-methoxyfuranocoumarin.